RNA 5'-cap (guanine-N7)-methylation [GO:0106005] (biological process) Definition: The process whereby a guanine in 5-cap is methylated at the N7 position of guanine. Sources: GOC:hjd Relationships: is a type of RNA (guanine-N7)-methylation [GO:0036265]; BFO_0000050 7-methylguanosine RNA capping [GO:0009452]